{
  "gene_symbol": "LYPD6B",
  "gene_name": "Ly6_PLAUR domain-containing protein 6B",
  "term_label": "Unknown biological process",
  "gene": "UniProtKB:Q8NI32",
  "term_id": "UNKNOWN:0002"
}